{
  "gene_symbol": "C22orf39",
  "gene_name": "UPF0545 protein C22orf39",
  "term_id": "UNKNOWN:0001",
  "term_label": "Unknown molecular function",
  "gene": "UniProtKB:Q6P5X5"
}